queuine import across plasma membrane [GO:0160284] (biological process) Definition: The directed movement of queuine from outside of a cell, across the plasma membrane and into the cytosol. Relationships: is a type of nitrogen compound transport [GO:0071705]; is a type of import across plasma membrane [GO:0098739] References: PMID:40526720